{
  "gene_name": "Arsenite methyltransferase",
  "gene": "UniProtKB:Q9HBK9",
  "term_id": "GO:0018872",
  "gene_symbol": "AS3MT",
  "term_label": "arsonoacetate metabolic process"
}